lumenal side of Golgi membrane [GO:0098547] (cellular component) Relationships: is a type of lumenal side of membrane [GO:0098576]; is part of Golgi membrane [GO:0000139] Sources: GOC:ab, GOC:dos Definition: The side of the Golgi membrane that faces the lumen.